{
  "term_id": "UNKNOWN:0001",
  "gene_name": "Integrator complex subunit 3",
  "term_label": "Unknown molecular function",
  "gene_symbol": "INTS3",
  "gene": "UniProtKB:Q68E01"
}